{
  "gene": "UniProtKB:Q6UXV3",
  "gene_symbol": "UNQ6126_PRO20091",
  "term_label": "Unknown biological process",
  "gene_name": "Uncharacterized protein UNQ6126_PRO20091",
  "term_id": "UNKNOWN:0002"
}